{
  "gene_symbol": "BTBD17",
  "gene_name": "BTB_POZ domain-containing protein 17",
  "gene": "UniProtKB:A6NE02",
  "term_id": "UNKNOWN:0003",
  "term_label": "Unknown cellular component"
}